{
  "gene_name": "Protein BUD31 homolog",
  "term_label": "mRNA splicing, via spliceosome",
  "term_id": "GO:0000398",
  "gene_symbol": "BUD31",
  "gene": "UniProtKB:P41223"
}